{
  "term_id": "UNKNOWN:0001",
  "term_label": "Unknown molecular function",
  "gene_name": "Interleukin-1 receptor-associated kinase 3",
  "gene": "UniProtKB:Q9Y616",
  "gene_symbol": "IRAK3"
}